{
  "gene": "UniProtKB:Q8TE02",
  "term_label": "elongator holoenzyme complex",
  "gene_symbol": "ELP5",
  "gene_name": "Elongator complex protein 5",
  "term_id": "GO:0033588"
}